{
  "gene_name": "Isopentenyl-diphosphate delta-isomerase 2",
  "term_label": "isopentenyl diphosphate biosynthetic process",
  "gene_symbol": "IDI2",
  "gene": "UniProtKB:Q9BXS1",
  "term_id": "GO:0009240"
}